glucocorticoid metabolic process [GO:0008211] (biological process) Sources: ISBN:0198506732 Regulation: RO_0002211 by regulation of glucocorticoid metabolic process [GO:0031943] Relationships: is a type of GO:0008202 Definition: The chemical reactions and pathways involving glucocorticoids, hormonal C21 corticosteroids synthesized from cholesterol. Glucocorticoids act primarily on carbohydrate and protein metabolism, and have anti-inflammatory effects. Also known as: glucocorticoid metabolism, glucocorticosteroid metabolic process, glucocorticosteroid metabolism Subtypes: glucocorticoid biosynthetic process [GO:0006704], glucocorticoid catabolic process [GO:0006713], cortisol metabolic process [GO:0034650]